negative regulation of tissue remodeling [GO:0034104] (biological process) Definition: Any process that stops, prevents, or reduces the frequency, rate, or extent of tissue remodeling. Also known as: negative regulation of tissue remodelling Relationships: is a type of regulation of tissue remodeling [GO:0034103]; is a type of negative regulation of multicellular organismal process [GO:0051241]; negatively regulates tissue remodeling [GO:0048771] Subtypes: negative regulation of erythrocyte clearance [GO:0034107], GO:0046851, negative regulation of blood vessel remodeling [GO:0060313], negative regulation of mammary gland involution [GO:1903520], negative regulation of connective tissue replacement [GO:1905204] Sources: GOC:add